{
  "gene": "UniProtKB:Q8TAM1",
  "gene_symbol": "BBS10",
  "term_id": "UNKNOWN:0003",
  "gene_name": "Bardet-Biedl syndrome 10 protein",
  "term_label": "Unknown cellular component"
}